{
  "term_id": "GO:0042626",
  "term_label": "ATPase-coupled transmembrane transporter activity",
  "gene_name": "ATP-binding cassette sub-family A member 13",
  "gene": "UniProtKB:Q86UQ4",
  "gene_symbol": "ABCA13"
}